maintenance of mitotic sister chromatid cohesion, arms [GO:0071959] (biological process) Definition: The process in which the association between sister chromatids of a replicated chromosome along the length of the chromosome arms, is maintained as chromosomes condense, attach to the spindle in a bipolar orientation, and congress to the metaphase plate during a mitotic cell cycle. References: PMID:1708436 Sources: GOC:mah Also known as: maintenance of mitotic sister chromatin cohesion along arms, maintenance of sister chromatin cohesion along arms at mitosis Relationships: is a type of GO:0034088; is part of mitotic sister chromatid cohesion, arms [GO:0071961] Regulation: RO_0002211 by regulation of maintenance of mitotic sister chromatid cohesion, arms [GO:2000715]; negatively regulated by negative regulation of maintenance of mitotic sister chromatid cohesion, arms [GO:2000716]; positively regulated by positive regulation of maintenance of mitotic sister chromatid cohesion, arms [GO:2000717]